{
  "term_id": "GO:0002456",
  "gene_name": "C4b-binding protein alpha chain",
  "gene_symbol": "C4BPA",
  "term_label": "T cell mediated immunity",
  "gene": "UniProtKB:P04003"
}